negative regulation of platelet rolling [GO:0160019] (biological process) References: PMID:15738422 Sources: GOC:sl, GO_REF:0000058 Relationships: is a type of negative regulation of heterotypic cell-cell adhesion [GO:0034115]; is a type of regulation of platelet rolling [GO:0160017]; negatively regulates platelet rolling [GO:0160015] Definition: Any process that decreases the rate, frequency, or extent of platelet rolling.